{
  "gene_symbol": "WDR55",
  "term_label": "Unknown cellular component",
  "gene": "UniProtKB:Q9H6Y2",
  "gene_name": "WD repeat-containing protein 55",
  "term_id": "UNKNOWN:0003"
}